{
  "term_id": "GO:0005886",
  "gene_symbol": "NOX5",
  "gene": "UniProtKB:Q96PH1",
  "gene_name": "NADPH oxidase 5",
  "term_label": "plasma membrane"
}